microvillar actin bundle [GO:0097516] (cellular component) Sources: GOC:cjm, GOC:mah Definition: A parallel bundle of actin filaments at the core of a microvillus. Relationships: is a type of actin filament bundle of actin-based cell projection [GO:0098859]; is part of microvillus [GO:0005902]